ADP-glyceromanno-heptose 6-epimerase activity [GO:0008712] (molecular function) Also known as: ADP-L-glycero-D-manno-heptose 6-epimerase activity, ADPglyceromanno-heptose 6-epimerase activity Relationships: is a type of racemase and epimerase activity, acting on carbohydrates and derivatives [GO:0016857] Sources: EC:5.1.3.20, RHEA:17577 Definition: Catalysis of the reaction: ADP-D-glycero-D-manno-heptose = ADP-L-glycero-D-manno-heptose.